regulation of mast cell cytokine production [GO:0032763] (biological process) Subtypes: negative regulation of mast cell cytokine production [GO:0032764], GO:0032765 Relationships: is a type of regulation of cytokine production involved in immune response [GO:0002718]; regulates mast cell cytokine production [GO:0032762] Sources: GOC:mah Definition: Any process that modulates the frequency, rate, or extent of mast cell cytokine production.